{
  "gene": "UniProtKB:P25391",
  "term_id": "UNKNOWN:0001",
  "gene_symbol": "LAMA1",
  "term_label": "Unknown molecular function",
  "gene_name": "Laminin subunit alpha-1"
}